{
  "gene_symbol": "GRID2",
  "gene": "UniProtKB:O43424",
  "term_id": "GO:0043197",
  "term_label": "dendritic spine",
  "gene_name": "Glutamate receptor ionotropic, delta-2"
}